cellular response to anisomycin [GO:0072740] (biological process) Sources: GOC:mah Definition: Any process that results in a change in state or activity of a cell (in terms of movement, secretion, enzyme production, gene expression, etc.) as a result of an anisomycin stimulus. Relationships: is a type of response to anisomycin [GO:0072739]